aspartoacylase activity [GO:0019807] (MF) Definition: Catalysis of the reaction: N-acyl-L-aspartate + H2O = a fatty acid anion + L-aspartate. Sources: EC:3.5.1.15 Relationships: is a type of GO:0016811 Also known as: N-acetylaspartate amidohydrolase activity, N-acyl-L-aspartate amidohydrolase activity, acetyl-aspartic deaminase activity, acylase II, aminoacylase II activity